determination of genital disc primordium [GO:0035225] (biological process) Definition: Allocation of embryonic cells to the genital imaginal disc founder populations. Early in development at the blastoderm stage, the anlage of the genital disc of both sexes consists of three primordia: the female genital primoridum lcoated anteriorly, the anal primoridum located posteriorly, and the male gential primordium between the two. References: PMID:11494318 Sources: GOC:bf Relationships: is a type of determination of imaginal disc primordium [GO:0007445]; is part of genital disc development [GO:0035215]